V1A vasopressin receptor binding [GO:0031894] (molecular function) Sources: GOC:mah, GOC:nln Definition: Binding to a V1A vasopressin receptor. Relationships: is a type of vasopressin receptor binding [GO:0031893] Also known as: V1A vasopressin receptor ligand